{
  "term_id": "GO:0016266",
  "term_label": "protein O-linked glycosylation via N-acetyl-galactosamine",
  "gene": "UniProtKB:Q8NBI6",
  "gene_name": "Xyloside xylosyltransferase 1",
  "gene_symbol": "XXYLT1"
}